{
  "gene_symbol": "C8orf58",
  "term_id": "UNKNOWN:0001",
  "term_label": "Unknown molecular function",
  "gene_name": "Uncharacterized protein C8orf58",
  "gene": "UniProtKB:Q8NAV2"
}